{
  "term_label": "protein import into mitochondrial matrix",
  "gene_name": "TOMM20-like protein 1",
  "term_id": "GO:0030150",
  "gene": "UniProtKB:Q6UXN7",
  "gene_symbol": "TOMM20L"
}